ovulation cycle [GO:0042698] (biological process) Subtypes: GO:0044849, GO:0044850 Definition: The type of sexual cycle seen in females, often with physiologic changes in the endometrium that recur at regular intervals during the reproductive years. Relationships: is a type of rhythmic process [GO:0048511]; is a type of multicellular organismal reproductive process [GO:0048609] Sources: ISBN:0721662544